{
  "term_id": "GO:0000785",
  "gene_name": "T-box transcription factor TBX20",
  "term_label": "chromatin",
  "gene_symbol": "TBX20",
  "gene": "UniProtKB:Q9UMR3"
}